excitation of vasomotor center by chemoreceptor signaling [GO:0002008] (biological process) Definition: The process in which the molecular signal from the carotid and aortic bodies is relayed to the vasomotor center, causing it to signal an increase arterial pressure. Sources: GOC:dph Also known as: excitation of vasomotor center by chemoreceptor signalling Relationships: is a type of nervous system process involved in regulation of systemic arterial blood pressure [GO:0001976]; is part of regulation of systemic arterial blood pressure by chemoreceptor signaling [GO:0001979]; is part of GO:0003084 Subtypes: excitation of vasomotor center by aortic body chemoreceptor signaling [GO:0003040], excitation of vasomotor center by carotid body chemoreceptor signaling [GO:0003041]